{
  "term_label": "Unknown molecular function",
  "term_id": "UNKNOWN:0001",
  "gene_name": "Protein SCO1 homolog, mitochondrial",
  "gene_symbol": "SCO1",
  "gene": "UniProtKB:O75880"
}